{
  "term_label": "signaling receptor activity",
  "term_id": "GO:0038023",
  "gene": "UniProtKB:Q8TF66",
  "gene_name": "Leucine-rich repeat-containing protein 15",
  "gene_symbol": "LRRC15"
}